{
  "gene": "UniProtKB:P22888",
  "term_id": "GO:0042700",
  "term_label": "luteinizing hormone signaling pathway",
  "gene_symbol": "LHCGR",
  "gene_name": "Lutropin-choriogonadotropic hormone receptor"
}